{
  "gene_symbol": "HES2",
  "term_id": "GO:0050767",
  "gene": "UniProtKB:Q9Y543",
  "gene_name": "Transcription factor HES-2",
  "term_label": "regulation of neurogenesis"
}